{
  "gene_symbol": "ITGA11",
  "term_label": "integrin alpha11-beta1 complex",
  "gene": "UniProtKB:Q9UKX5",
  "gene_name": "Integrin alpha-11",
  "term_id": "GO:0034681"
}